{
  "term_label": "phototransduction",
  "gene": "UniProtKB:Q9NP86",
  "gene_symbol": "CABP5",
  "term_id": "GO:0007602",
  "gene_name": "Calcium-binding protein 5"
}